geranylgeranyl reductase activity [GO:0045550] (molecular function) Definition: Catalysis of the formation of phytyl group from the stepwise reduction of a geranylgeranyl group. Relationships: is a type of GO:0016491 References: PMID:9492312